meiotic centromere clustering [GO:1990571] (biological process) References: PMID:10366596, PMID:9009280 Relationships: is a type of meiotic chromosome movement towards spindle pole [GO:0016344]; is a type of chromosome organization involved in meiotic cell cycle [GO:0070192]; is a type of centromere clustering [GO:0098653] Also known as: centromere clustering during meiosis, homologous chromosome movement towards spindle pole in meiosis I prometaphase Definition: The process by which centromeres/kinetochores attach to and migrate along microtubules to become localized to clusters at the spindle pole body during a meiotic prometaphase I.